cerebellar molecular layer development [GO:0021679] (biological process) Definition: The process whose specific outcome is the progression of the cerebellar molecular layer nerve over time, from its formation to the mature structure. The molecular layer is the outermost layer of the cerebellar cortex. It contains the parallel fibers of the granule cells, interneurons such as stellate and basket cells, and the dendrites of the underlying Purkinje cells. Relationships: is a type of anatomical structure development [GO:0048856]; is part of GO:0021695 Sources: GOC:cls, GOC:dgh, GOC:dph, GOC:jid, GO_REF:0000021